{
  "term_id": "GO:0008889",
  "gene_name": "Glycerophosphodiester phosphodiesterase domain-containing protein 4",
  "gene": "UniProtKB:Q6W3E5",
  "term_label": "glycerophosphodiester phosphodiesterase activity",
  "gene_symbol": "GDPD4"
}